spitzenkorper [GO:0031521] (cellular component) Definition: Structure within the hyphal tip of filamentous fungi that acts as an organizing center for hyphal tip growth; may function to supply vesicles to the elongating tip and/or to organize cytoskeletal microfilaments. References: PMID:15701784, PMID:15976451 Relationships: is a type of protein-containing complex [GO:0032991]; is part of hyphal tip [GO:0001411]; is part of GO:0012505